{
  "term_id": "GO:0005737",
  "gene_symbol": "PUM2",
  "gene_name": "Pumilio homolog 2",
  "term_label": "cytoplasm",
  "gene": "UniProtKB:Q8TB72"
}